{
  "term_label": "DNA cytosine deamination",
  "gene_name": "Single-stranded DNA cytosine deaminase",
  "gene": "UniProtKB:Q9GZX7",
  "term_id": "GO:0070383",
  "gene_symbol": "AICDA"
}